{
  "term_id": "UNKNOWN:0003",
  "term_label": "Unknown cellular component",
  "gene_symbol": "C12orf57",
  "gene_name": "Protein C10",
  "gene": "UniProtKB:Q99622"
}